{
  "gene": "UniProtKB:Q9BQ66",
  "gene_name": "Keratin-associated protein 4-12",
  "term_id": "UNKNOWN:0001",
  "gene_symbol": "KRTAP4-12",
  "term_label": "Unknown molecular function"
}